positive regulation of cardiac muscle cell differentiation [GO:2000727] (biological process) Sources: GOC:BHF Also known as: positive regulation of cardiomyocyte differentiation, positive regulation of heart muscle cell differentiation Subtypes: positive regulation of cardiac muscle fiber development [GO:0055020] Definition: Any process that activates or increases the frequency, rate or extent of cardiac muscle cell differentiation. Relationships: is a type of GO:0051155; is a type of GO:1905209; is a type of regulation of cardiac muscle cell differentiation [GO:2000725]; positively regulates cardiac muscle cell differentiation [GO:0055007]